{
  "term_label": "RNA polymerase I complex",
  "gene": "UniProtKB:Q9GZS1",
  "gene_name": "DNA-directed RNA polymerase I subunit RPA49",
  "term_id": "GO:0005736",
  "gene_symbol": "POLR1E"
}